{
  "term_label": "regulation of immune system process",
  "gene_symbol": "ZBTB14",
  "gene_name": "Zinc finger and BTB domain-containing protein 14",
  "term_id": "GO:0002682",
  "gene": "UniProtKB:O43829"
}